{
  "gene_name": "Zinc finger protein 675",
  "gene_symbol": "ZNF675",
  "term_id": "GO:0000978",
  "gene": "UniProtKB:Q8TD23",
  "term_label": "RNA polymerase II cis-regulatory region sequence-specific DNA binding"
}